{
  "gene_name": "Centrosomal protein of 72 kDa",
  "gene": "UniProtKB:Q9P209",
  "gene_symbol": "CEP72",
  "term_label": "spindle organization",
  "term_id": "GO:0007051"
}